{
  "gene_name": "Nuclear protein 1",
  "gene": "UniProtKB:O60356",
  "term_id": "UNKNOWN:0001",
  "term_label": "Unknown molecular function",
  "gene_symbol": "NUPR1"
}